{
  "gene_name": "Nuclear distribution protein nudE-like 1",
  "term_id": "GO:0007100",
  "gene_symbol": "NDEL1",
  "term_label": "mitotic centrosome separation",
  "gene": "UniProtKB:Q9GZM8"
}